{
  "gene": "UniProtKB:Q7Z3S9",
  "term_label": "Unknown biological process",
  "gene_symbol": "NOTCH2NLA",
  "gene_name": "Notch homolog 2 N-terminal-like protein A",
  "term_id": "UNKNOWN:0002"
}